{
  "gene_name": "Adhesion G-protein coupled receptor G1",
  "gene": "UniProtKB:Q9Y653",
  "term_id": "GO:0005886",
  "gene_symbol": "ADGRG1",
  "term_label": "plasma membrane"
}